{
  "term_label": "serine-type endopeptidase activity",
  "gene": "UniProtKB:P00750",
  "term_id": "GO:0004252",
  "gene_name": "Tissue-type plasminogen activator",
  "gene_symbol": "PLAT"
}